negative regulation of phospholipid transport [GO:2001139] (BP) Definition: Any process that stops, prevents or reduces the frequency, rate or extent of phospholipid transport. Relationships: is a type of negative regulation of lipid transport [GO:0032369]; is a type of GO:2001138; RO_0002212 GO:0015914 Subtypes: negative regulation of phospholipid translocation [GO:0061093], negative regulation of phospholipid efflux [GO:1902999] Sources: GOC:obol